{
  "gene_name": "Uncharacterized protein KIAA2012",
  "term_id": "UNKNOWN:0003",
  "gene": "UniProtKB:Q0VF49",
  "gene_symbol": "KIAA2012",
  "term_label": "Unknown cellular component"
}